maintenance of epithelial cell apical/basal polarity [GO:0045199] (biological process) Relationships: is a type of maintenance of apical/basal cell polarity [GO:0035090]; is a type of GO:0045197 Sources: GOC:bf Definition: The maintenance of the apicobasal polarity of an epithelial cell.